{
  "gene_symbol": "WFDC13",
  "term_id": "GO:0019731",
  "gene": "UniProtKB:Q8IUB5",
  "gene_name": "WAP four-disulfide core domain protein 13",
  "term_label": "antibacterial humoral response"
}